{
  "gene": "UniProtKB:P29371",
  "gene_name": "Neuromedin-K receptor",
  "term_id": "GO:0097225",
  "term_label": "sperm midpiece",
  "gene_symbol": "TACR3"
}